axis elongation involved in somitogenesis [GO:0090245] (biological process) Sources: GOC:ascb_2009, GOC:dph, GOC:tb Relationships: is a type of axis elongation [GO:0003401]; BFO_0000050 somitogenesis [GO:0001756] Definition: The developmental growth that results in the elongation of the rostral-caudal axis that contributes to somitogenesis.